regulation of primary cell septum biogenesis [GO:1905756] (biological process) Definition: Any process that modulates the frequency, rate or extent of primary cell septum biogenesis. References: PMID:27898700 Sources: GOC:TermGenie, GO_REF:0000058 Relationships: is a type of GO:0140279; RO_0002211 GO:0031671 Subtypes: negative regulation of primary cell septum biogenesis [GO:1905757], GO:1905758